{
  "term_label": "acetylcholine catabolic process",
  "term_id": "GO:0006581",
  "gene_name": "Cholinesterase",
  "gene_symbol": "BCHE",
  "gene": "UniProtKB:P06276"
}